cytogamy [GO:0000755] (biological process) Sources: GOC:elh Definition: During conjugation with cellular fusion, the process resulting in creating a single cell from complementary mating types. The localized remodeling and dissolution of external protective structures allow the fusion of the plasma membranes and cytoplasmic mixing. An example of this process is found in Saccharomyces cerevisiae. Also known as: zygote formation Relationships: is a type of GO:0022413; is part of GO:0000747